{
  "gene_name": "Casein kinase II subunit alpha'",
  "term_id": "GO:0005956",
  "gene_symbol": "CSNK2A2",
  "term_label": "protein kinase CK2 complex",
  "gene": "UniProtKB:P19784"
}